{
  "gene_name": "Forkhead box protein E3",
  "term_label": "Unknown cellular component",
  "gene": "UniProtKB:Q13461",
  "term_id": "UNKNOWN:0003",
  "gene_symbol": "FOXE3"
}